{
  "gene_name": "Ret finger protein-like 3",
  "gene": "UniProtKB:O75679",
  "term_label": "innate immune response",
  "term_id": "GO:0045087",
  "gene_symbol": "RFPL3"
}